{
  "gene_symbol": "Q6JHZ5",
  "term_label": "Unknown molecular function",
  "term_id": "UNKNOWN:0001",
  "gene": "UniProtKB:Q6JHZ5",
  "gene_name": "NS5ATP13TP1"
}